{
  "gene": "UniProtKB:Q86UB9",
  "term_id": "UNKNOWN:0003",
  "term_label": "Unknown cellular component",
  "gene_symbol": "TMEM135",
  "gene_name": "Transmembrane protein 135"
}